negative regulation of aeciospore formation [GO:0075250] (biological process) Relationships: is a type of negative regulation of asexual sporulation resulting in formation of a cellular spore [GO:0043944]; is a type of regulation of aeciospore formation [GO:0075248]; negatively regulates aeciospore formation [GO:0075247] Sources: GOC:pamgo_curators Definition: Any process that stops, prevents, or reduces the frequency, rate or extent of aeciospore formation, a process in which a dikaryotic spore of typically a rust fungus is produced in an aecium.